{
  "gene_symbol": "ZPLD1",
  "gene_name": "Zona pellucida-like domain-containing protein 1",
  "gene": "UniProtKB:Q8TCW7",
  "term_id": "GO:0009986",
  "term_label": "cell surface"
}